{
  "term_id": "GO:0007189",
  "term_label": "adenylate cyclase-activating G protein-coupled receptor signaling pathway",
  "gene_symbol": "PTH1R",
  "gene_name": "Parathyroid hormone_parathyroid hormone-related peptide receptor",
  "gene": "UniProtKB:Q03431"
}